positive regulation of hormone metabolic process [GO:0032352] (biological process) Subtypes: positive regulation of juvenile hormone catabolic process [GO:0045971], positive regulation of hormone biosynthetic process [GO:0046886], GO:0060569, positive regulation of auxin metabolic process [GO:0090355], positive regulation of retinoic acid biosynthetic process [GO:1900054], GO:2000488, positive regulation of thyroid hormone generation [GO:2000611] Also known as: positive regulation of hormone metabolism, up regulation of hormone metabolic process, up-regulation of hormone metabolic process, upregulation of hormone metabolic process, activation of hormone metabolic process, stimulation of hormone metabolic process Definition: Any process that activates or increases the frequency, rate or extent of the chemical reactions and pathways involving any hormone. Relationships: is a type of positive regulation of metabolic process [GO:0009893]; is a type of regulation of hormone metabolic process [GO:0032350]; positively regulates hormone metabolic process [GO:0042445] Sources: GOC:mah